{
  "gene": "UniProtKB:Q9NSI6",
  "term_id": "GO:0007010",
  "gene_name": "Bromodomain and WD repeat-containing protein 1",
  "term_label": "cytoskeleton organization",
  "gene_symbol": "BRWD1"
}